{
  "gene": "UniProtKB:Q969K7",
  "term_id": "UNKNOWN:0002",
  "gene_name": "Transmembrane protein 54",
  "gene_symbol": "TMEM54",
  "term_label": "Unknown biological process"
}